D-lysine catabolic process [GO:0019476] (biological process) Also known as: D-lysine breakdown, D-lysine catabolism, D-lysine degradation Relationships: is a type of lysine catabolic process [GO:0006554]; is a type of D-amino acid catabolic process [GO:0019478] Sources: GOC:ai, GOC:jsg, GOC:mah Definition: The chemical reactions and pathways resulting in the breakdown of D-lysine, the D-enantiomer of lysine; i.e. (2R)-2,6-diaminohexanoic acid.